{
  "gene_name": "Zinc finger protein 878",
  "gene_symbol": "ZNF878",
  "gene": "UniProtKB:C9JN71",
  "term_id": "GO:0000977",
  "term_label": "RNA polymerase II transcription regulatory region sequence-specific DNA binding"
}